IgM binding [GO:0001791] (molecular function) Definition: Binding to an immunoglobulin of the IgM isotype. Sources: GOC:add, ISBN:0781735149 Relationships: is a type of immunoglobulin binding [GO:0019865]